{
  "gene": "UniProtKB:P21917",
  "gene_symbol": "DRD4",
  "term_label": "G protein-coupled receptor signaling pathway, coupled to cyclic nucleotide second messenger",
  "term_id": "GO:0007187",
  "gene_name": "D(4) dopamine receptor"
}